{
  "gene_symbol": "SCGN",
  "gene_name": "Secretagogin",
  "term_id": "GO:0005634",
  "gene": "UniProtKB:O76038",
  "term_label": "nucleus"
}